{
  "gene_symbol": "A0A5F9ZGZ6",
  "gene": "UniProtKB:A0A5F9ZGZ6",
  "gene_name": "Rho guanine nucleotide exchange factor 5_35 N-terminal domain-containing protein",
  "term_id": "UNKNOWN:0001",
  "term_label": "Unknown molecular function"
}